{
  "term_id": "GO:0003785",
  "gene_name": "Thymosin beta-15B",
  "term_label": "actin monomer binding",
  "gene_symbol": "TMSB15B",
  "gene": "UniProtKB:P0CG35"
}